ABC-type taurine transporter transporter activity [GO:0015411] (molecular function) Relationships: is a type of taurine transmembrane transporter activity [GO:0005368]; is a type of ABC-type alkanesulfonate transporter transporter activity [GO:0042959] Also known as: taurine ABC transporter, ATP-dependent taurine transporter activity, ATPase-coupled taurine transporter activity, taurine-transporting ATPase activity Sources: RHEA:14613 Definition: Enables the transfer of taurine from one side of a membrane to the other according to the reaction: ATP + H2O + taurine(out) = ADP + phosphate + taurine(in).